{
  "gene": "UniProtKB:Q9Y279",
  "gene_name": "V-set and immunoglobulin domain-containing protein 4",
  "term_id": "GO:0042130",
  "gene_symbol": "VSIG4",
  "term_label": "negative regulation of T cell proliferation"
}